{
  "gene_name": "Pre-B-cell leukemia transcription factor 3",
  "gene_symbol": "PBX3",
  "gene": "UniProtKB:P40426",
  "term_id": "GO:0005634",
  "term_label": "nucleus"
}